{
  "gene_symbol": "SYNPR",
  "gene": "UniProtKB:Q8TBG9",
  "term_id": "UNKNOWN:0001",
  "gene_name": "Synaptoporin",
  "term_label": "Unknown molecular function"
}